tRNA exon ligation [GO:0000968] (BP) Definition: An RNA exon ligation process that rejoins two exons of a pre-tRNA which has had the intron removed. Relationships: is a type of RNA exon ligation [GO:0000378]; is part of tRNA splicing, via endonucleolytic cleavage and ligation [GO:0006388] Sources: GOC:krc